{
  "gene": "UniProtKB:Q32M88",
  "gene_symbol": "PGGHG",
  "gene_name": "Protein-glucosylgalactosylhydroxylysine glucosidase",
  "term_label": "cytosol",
  "term_id": "GO:0005829"
}